{
  "term_id": "GO:0005737",
  "gene_name": "Serine_threonine-protein kinase MARK2",
  "term_label": "cytoplasm",
  "gene": "UniProtKB:Q7KZI7",
  "gene_symbol": "MARK2"
}